regulation of cAMP-dependent protein kinase activity [GO:2000479] (biological process) Sources: GOC:obol Definition: Any process that modulates the frequency, rate or extent of cAMP-dependent protein kinase activity. Relationships: is_a GO:0071900; regulates cAMP-dependent protein kinase activity [GO:0004691] Subtypes: negative regulation of cAMP-dependent protein kinase activity [GO:2000480], positive regulation of cAMP-dependent protein kinase activity [GO:2000481] Also known as: regulation of 3',5' cAMP-dependent protein kinase activity, regulation of 3',5'-cAMP-dependent protein kinase activity, regulation of ATP:protein phosphotransferase (cAMP-dependent) activity, regulation of adenosine 3',5'-cyclophosphate-dependent protein kinase activity, regulation of cAMP-dependent protein kinase, intrinsic catalyst activity, regulation of cyclic AMP-dependent protein kinase activity, regulation of AMPK, regulation of PKA, regulation of PKA C, regulation of STK22, regulation of protein kinase A activity